{
  "term_id": "GO:0005768",
  "term_label": "endosome",
  "gene_name": "Ras-related protein Rab-40B",
  "gene": "UniProtKB:Q12829",
  "gene_symbol": "RAB40B"
}